{
  "gene_symbol": "GRK7",
  "gene_name": "Rhodopsin kinase GRK7",
  "term_label": "regulation of signal transduction",
  "term_id": "GO:0009966",
  "gene": "UniProtKB:Q8WTQ7"
}